hexaprenyl-diphosphate synthase ((2E,6E)-farnesyl-diphosphate specific) activity [GO:0036423] (molecular function) Sources: RHEA:27559 Definition: Catalysis of the reaction: (2E,6E)-farnesyl diphosphate + 3 isopentenyl diphosphate = 3 diphosphate + all-trans-hexaprenyl diphosphate. Also known as: hexaprenyl diphosphate synthase activity, hexaprenyl pyrophosphate synthetase activity, HexPS activity Relationships: is a type of GO:0120531